{
  "term_label": "G protein-coupled serotonin receptor activity",
  "gene_name": "5-hydroxytryptamine receptor 1E",
  "term_id": "GO:0004993",
  "gene_symbol": "HTR1E",
  "gene": "UniProtKB:P28566"
}